{
  "gene": "UniProtKB:Q14929",
  "gene_symbol": "ZNF169",
  "gene_name": "Zinc finger protein 169",
  "term_label": "DNA-binding transcription factor activity, RNA polymerase II-specific",
  "term_id": "GO:0000981"
}